positive regulation of hypoxanthine transport [GO:0035346] (biological process) Relationships: is a type of positive regulation of nucleobase-containing compound transport [GO:0032241]; is a type of regulation of hypoxanthine transport [GO:0035345]; positively regulates GO:0035344 Sources: GOC:bf Also known as: positive regulation of 6-hydroxypurine transport Definition: Any process that activates or increases the frequency, rate or extent of the directed movement of hypoxanthine into, out of or within a cell, or between cells, by means of some agent such as a transporter or pore.